{
  "term_id": "UNKNOWN:0001",
  "term_label": "Unknown molecular function",
  "gene": "UniProtKB:Q8WXH5",
  "gene_name": "Suppressor of cytokine signaling 4",
  "gene_symbol": "SOCS4"
}